regulation of trans-synaptic signaling by endocannabinoid, modulating synaptic transmission [GO:0150036] (biological process) References: PMID:27296803 Sources: GOC:aruk, GOC:bc Definition: Any process that modulates the frequency, rate or extent of trans-synaptic signaling by endocannabinoid, modulating synaptic transmission. Relationships: is a type of modulation of chemical synaptic transmission [GO:0050804]; regulates GO:0099553 Note: Note that this term was created for the SynGO project, and will be obsoleted when the SynGO annotations are made in Noctua.